3',2'-cyclic GMP-AMP binding [GO:0140704] (molecular function) Definition: Binding to 3',2' cyclic GMP-AMP (cGAMP) nucleotide, a cyclic purine dinucleotide that consists of AMP and GMP units cyclized via 3',5' and 2',5' linkages. References: PMID:34261127 Also known as: 3',2' cyclic-GMP-AMP binding, 3',2'-cGAMP binding, 3',2'-cyclic GAMP binding Relationships: is a type of anion binding [GO:0043168]